L-amino-acid alpha-ligase activity [GO:0034026] (molecular function) Relationships: is a type of acid-amino acid ligase activity [GO:0016881] Also known as: L-amino acid alpha-ligase activity, L-amino acid ligase activity, bacilysin synthetase activity, YwfE Sources: EC:6.3.2.49 Definition: Catalysis of the reaction: ATP + an L-amino acid + an L-amino acid = ADP + phosphate + L-aminoacyl-L-amino acid.